{
  "gene": "UniProtKB:Q8NGJ8",
  "term_id": "GO:0004984",
  "gene_name": "Olfactory receptor 51S1",
  "gene_symbol": "OR51S1",
  "term_label": "olfactory receptor activity"
}